cleavage in ITS2 between 5.8S rRNA and LSU-rRNA of tricistronic rRNA transcript (SSU-rRNA, 5.8S rRNA, LSU-rRNA) [GO:0000448] (biological process) References: PMID:10690410 Sources: GOC:curators Relationships: is a type of endonucleolytic cleavage of tricistronic rRNA transcript (SSU-rRNA, 5.8S rRNA, LSU-rRNA) [GO:0000479]; is part of maturation of LSU-rRNA from tricistronic rRNA transcript (SSU-rRNA, 5.8S rRNA, LSU-rRNA) [GO:0000463]; is part of maturation of 5.8S rRNA from tricistronic rRNA transcript (SSU-rRNA, 5.8S rRNA, LSU-rRNA) [GO:0000466] Also known as: cleavage in ITS2 of tricistronic rRNA transcript to separate 5.8S and LSU rRNAs (SSU-rRNA, 5.8S rRNA, LSU-rRNA), cleavage at C2 Definition: Endonucleolytic cleavage within ITS2 between the 5.8S rRNA and the LSU-rRNA of an rRNA molecule originally produced as a tricistronic rRNA transcript that contained the Small SubUnit (SSU) rRNA, the 5.8S rRNA, and the Large SubUnit (LSU) rRNA, in that order, from 5' to 3' along the primary transcript.